negative regulation of tendon cell differentiation [GO:2001050] (biological process) Sources: GOC:obol Also known as: negative regulation of muscle attachment cell differentiation, negative regulation of tenocyte differentiation Relationships: is a type of negative regulation of cell differentiation [GO:0045596]; is a type of regulation of tendon cell differentiation [GO:2001049]; negatively regulates tendon cell differentiation [GO:0035990] Definition: Any process that stops, prevents or reduces the frequency, rate or extent of tendon cell differentiation.